{
  "gene_name": "Excitatory amino acid transporter 3",
  "gene": "UniProtKB:P43005",
  "gene_symbol": "SLC1A1",
  "term_label": "plasma membrane",
  "term_id": "GO:0005886"
}